{
  "term_id": "GO:0005794",
  "gene_name": "Bifunctional heparan sulfate N-deacetylase_N-sulfotransferase 2",
  "gene_symbol": "NDST2",
  "term_label": "Golgi apparatus",
  "gene": "UniProtKB:P52849"
}